{
  "gene_symbol": "OR14A2",
  "gene": "UniProtKB:Q96R54",
  "term_id": "GO:0004984",
  "term_label": "olfactory receptor activity",
  "gene_name": "Olfactory receptor 14A2"
}